{
  "gene_name": "Protein BUD31 homolog",
  "term_id": "GO:0005681",
  "gene_symbol": "BUD31",
  "gene": "UniProtKB:P41223",
  "term_label": "spliceosomal complex"
}